{
  "gene": "UniProtKB:Q15303",
  "term_id": "GO:0030182",
  "gene_name": "Receptor tyrosine-protein kinase erbB-4",
  "term_label": "neuron differentiation",
  "gene_symbol": "ERBB4"
}